{
  "term_label": "ubiquitin protein ligase activity",
  "gene": "UniProtKB:Q5U5R9",
  "gene_name": "Probable E3 ubiquitin-protein ligase HECTD2",
  "gene_symbol": "HECTD2",
  "term_id": "GO:0061630"
}